nucleus accumbens development [GO:0021768] (biological process) Sources: GOC:cls, GOC:dgh, GOC:dph, GOC:jid, GO_REF:0000021 Relationships: is a type of neural nucleus development [GO:0048857]; is part of striatum development [GO:0021756]; is part of GO:0021761 Also known as: ventral striatum development, accumbens nucleus development Definition: The progression of the nucleus accumbens over time from its initial formation until its mature state. The nucleus accumbens is a collection of pleomorphic cells in the caudal part of the anterior horn of the lateral ventricle, in the region of the olfactory tubercle, lying between the head of the caudate nucleus and the anterior perforated substance. It is part of the ventral striatum, a composite structure considered part of the basal ganglia.